sporocyte differentiation [GO:0048533] (biological process) Sources: GOC:tair_curators Subtypes: microsporocyte differentiation [GO:0010480], GO:1904159 Relationships: is a type of cell differentiation [GO:0030154] Also known as: sporocyte development, sporocyte morphogenesis Definition: The process in which a relatively unspecialized floral cell acquires the specialized features of a sporocyte. Sporocytes are the haploid spores of angiosperms. Once formed, they undergo meiotic divisions to form microspores and megaspores.